{
  "gene": "UniProtKB:A0A075B6W7",
  "term_id": "UNKNOWN:0001",
  "gene_name": "T cell receptor alpha joining 38 (Fragment)",
  "term_label": "Unknown molecular function",
  "gene_symbol": "TRAJ38"
}